benzoyl acetate-CoA ligase activity [GO:0018856] (molecular function) Definition: Catalysis of the reaction: 3-oxo-3-phenylpropionate + CoA + ATP = AMP + diphosphate + benzoyl acetyl-CoA. Relationships: is a type of CoA-ligase activity [GO:0016405]; is a type of acid-thiol ligase activity [GO:0016878] Sources: UM-BBD_reactionID:r0242